{
  "term_label": "DNA replication initiation",
  "gene_name": "DNA replication licensing factor MCM5",
  "term_id": "GO:0006270",
  "gene": "UniProtKB:P33992",
  "gene_symbol": "MCM5"
}